{
  "term_id": "GO:0000981",
  "gene_symbol": "DMRT2",
  "term_label": "DNA-binding transcription factor activity, RNA polymerase II-specific",
  "gene_name": "Doublesex- and mab-3-related transcription factor 2",
  "gene": "UniProtKB:Q9Y5R5"
}